{
  "term_label": "double-stranded DNA binding",
  "gene_symbol": "SYCP1",
  "gene": "UniProtKB:Q15431",
  "term_id": "GO:0003690",
  "gene_name": "Synaptonemal complex protein 1"
}